pancreatic juice secretion [GO:0030157] (biological process) Definition: The regulated release of pancreatic juice by the exocrine pancreas into the upper part of the intestine. Pancreatic juice is slightly alkaline and contains numerous enzymes and inactive enzyme precursors including alpha-amylase, chymotrypsinogen, lipase, procarboxypeptidase, proelastase, prophospholipase A2, ribonuclease, and trypsinogen. Its high concentration of bicarbonate ions helps to neutralize the acid from the stomach. Relationships: is a type of body fluid secretion [GO:0007589]; is a type of GO:0022600; is a type of secretion by tissue [GO:0032941] Regulation: regulated by regulation of pancreatic juice secretion [GO:0090186]; positively regulated by positive regulation of pancreatic juice secretion [GO:0090187]; negatively regulated by negative regulation of pancreatic juice secretion [GO:0090188] Sources: GOC:mah, ISBN:0198506732